negative regulation of matrix metallopeptidase secretion [GO:1904465] (biological process) References: PMID:8679543 Sources: GOC:TermGenie, GO_REF:0000058 Also known as: down regulation of MMP secretion, down regulation of matrix metallopeptidase secretion, down-regulation of MMP secretion, down-regulation of matrix metallopeptidase secretion, downregulation of MMP secretion, downregulation of matrix metallopeptidase secretion, negative regulation of MMP secretion, down regulation of matrix metalloproteinase secretion, down-regulation of matrix metalloproteinase secretion, downregulation of matrix metalloproteinase secretion, inhibition of MMP secretion, inhibition of matrix metallopeptidase secretion, inhibition of matrix metalloproteinase secretion, negative regulation of matrix metalloproteinase secretion Definition: Any process that stops, prevents or reduces the frequency, rate or extent of matrix metallopeptidase secretion. Relationships: is a type of negative regulation of protein secretion [GO:0050709]; is_a regulation of matrix metallopeptidase secretion [GO:1904464]; negatively regulates matrix metallopeptidase secretion [GO:1990773]